{
  "term_id": "UNKNOWN:0002",
  "gene_name": "Adenylate kinase isoenzyme 5",
  "term_label": "Unknown biological process",
  "gene_symbol": "AK5",
  "gene": "UniProtKB:Q9Y6K8"
}